{
  "gene": "UniProtKB:P11309",
  "gene_name": "Serine_threonine-protein kinase pim-1",
  "gene_symbol": "PIM1",
  "term_id": "GO:0007346",
  "term_label": "regulation of mitotic cell cycle"
}